{
  "gene_name": "PACRG-like protein",
  "term_id": "UNKNOWN:0001",
  "gene": "UniProtKB:Q8N7B6",
  "gene_symbol": "PACRGL",
  "term_label": "Unknown molecular function"
}